{
  "gene_name": "Aflatoxin B1 aldehyde reductase member 4",
  "term_id": "UNKNOWN:0002",
  "term_label": "Unknown biological process",
  "gene": "UniProtKB:Q8NHP1",
  "gene_symbol": "AKR7L"
}